{
  "gene": "UniProtKB:Q7Z745",
  "term_id": "GO:0001669",
  "term_label": "acrosomal vesicle",
  "gene_name": "Maestro heat-like repeat-containing protein family member 2B",
  "gene_symbol": "MROH2B"
}